histone H3T6 kinase activity [GO:0035403] (molecular function) Definition: Catalysis of the reaction: histone H3-threonine (position 6) + ATP = histone H3-phosphothreonine (position 6) + ADP. This reaction is the addition of a phosphate group to the threonine residue at position 6 of histone H3. Sources: GOC:bf Note: Comment: Note that the residue position corresponds to the canonical human H3 histone (UniProtKB:P84243); this residue is conserved across all eukaryotes. Residue 1 is the first residue following removal of the initiating Methionine (Met). Note that each histone is encoded by multiple genes, and sequences may vary across different genes within an organism. Relationships: is a type of GO:0004674; is a type of GO:0140996 Also known as: histone H3-T6 kinase activity, histone kinase activity (H3-T6 specific), histone threonine kinase activity (H3-T6 specific), histone-threonine kinase activity (H3-T6 specific)